{
  "gene_name": "Methionine-R-sulfoxide reductase B3",
  "gene": "UniProtKB:Q8IXL7",
  "gene_symbol": "MSRB3",
  "term_id": "GO:0033743",
  "term_label": "peptide-methionine (R)-S-oxide reductase activity"
}